{
  "gene_symbol": "TNFSF10",
  "gene": "UniProtKB:P50591",
  "gene_name": "Tumor necrosis factor ligand superfamily member 10",
  "term_id": "GO:0005125",
  "term_label": "cytokine activity"
}